bacterial-type flagellum basal body, C ring [GO:0009433] (cellular component) Definition: Cytoplasmic ring located at the base of the bacterial-type flagellar basal body; acts as a rotor; includes three switch proteins, which generate torque and can change their conformational state in a bimodal fashion, so that the motor direction can switch between clockwise and counterclockwise. Relationships: is a type of GO:0110165; is part of bacterial-type flagellum basal body [GO:0009425] References: PMID:10572114, PMID:12624192 Sources: GOC:cilia, GOC:mtg_sensu Also known as: flagellar basal body, C ring, flagellin-based flagellum basal body, C ring